{
  "gene_name": "Alpha-1A adrenergic receptor",
  "gene": "UniProtKB:P35348",
  "term_label": "positive regulation of cytosolic calcium ion concentration",
  "term_id": "GO:0007204",
  "gene_symbol": "ADRA1A"
}